euchromatin-nuclear membrane anchor activity [GO:0062240] (molecular function) Also known as: euchromatin-nuclear membrane tether activity, nuclear membrane-euchromatin anchor activity, nuclear membrane-euchromatin tether activity Definition: Binding to euchromatin and the nuclear inner membrane, in order to establish and maintain the euchromatin location and organization. References: PMID:31635174 Relationships: is a type of chromatin-nuclear membrane anchor activity [GO:0140707]